{
  "gene": "UniProtKB:P50897",
  "term_label": "lysosome",
  "gene_symbol": "PPT1",
  "term_id": "GO:0005764",
  "gene_name": "Palmitoyl-protein thioesterase 1"
}